phenylpyruvate tautomerase activity [GO:0050178] (molecular function) Definition: Catalysis of the reaction: keto-phenylpyruvate = enol-phenylpyruvate. Sources: RHEA:17097 Also known as: phenylpyruvate keto--enol tautomerase activity, phenylpyruvate keto-enol-isomerase activity, phenylpyruvic keto--enol isomerase activity Relationships: is a type of intramolecular oxidoreductase activity, interconverting keto- and enol-groups [GO:0016862]